negative regulation of post-translational protein targeting to membrane, translocation [GO:0120236] (biological process) Definition: Any process that stops, prevents or reduces the frequency, rate or extent of posttranslational protein translocation through the ER membrane. References: PMID:32513868 Sources: GOC:krc, GOC:rn Also known as: negative regulation of posttranslational endoplasmic reticulum membrane protein translocation, negative regulation of posttranslational protein targeting to membrane, translocation, negative regulation of N-terminal signal peptide-independent translocation into the ER, negative regulation of SRP-independent endoplasmic reticulum protein-membrane targeting, translocation Relationships: is a type of GO:0034763; is_a negative regulation of intracellular protein transport [GO:0090317]; is a type of regulation of post-translational protein targeting to membrane, translocation [GO:0120235]; negatively regulates GO:0031204